response to amine [GO:0014075] (biological process) Definition: Any process that results in a change in state or activity of a cell or an organism (in terms of movement, secretion, enzyme production, gene expression, etc.) as a result of an amine stimulus. An amine is a compound formally derived from ammonia by replacing one, two or three hydrogen atoms by hydrocarbyl groups. Subtypes: response to amphetamine [GO:0001975], response to methylamine [GO:0036255], GO:0071418, response to hesperadin [GO:1901595], GO:1901905, response to methamphetamine hydrochloride [GO:1904313] Sources: GOC:ef Also known as: response to amine stimulus Relationships: is a type of GO:1901698